{
  "gene_symbol": "HERC1",
  "term_id": "UNKNOWN:0001",
  "gene_name": "Probable E3 ubiquitin-protein ligase HERC1",
  "term_label": "Unknown molecular function",
  "gene": "UniProtKB:Q15751"
}